{
  "term_id": "GO:0031145",
  "gene": "UniProtKB:Q12834",
  "gene_name": "Cell division cycle protein 20 homolog",
  "term_label": "anaphase-promoting complex-dependent catabolic process",
  "gene_symbol": "CDC20"
}